{
  "gene_symbol": "SPON1",
  "gene": "UniProtKB:Q9HCB6",
  "gene_name": "Spondin-1",
  "term_label": "extracellular matrix",
  "term_id": "GO:0031012"
}